{
  "gene_symbol": "IL11RA",
  "gene": "UniProtKB:Q14626",
  "gene_name": "Interleukin-11 receptor subunit alpha",
  "term_label": "receptor complex",
  "term_id": "GO:0043235"
}